{
  "term_id": "GO:0005829",
  "term_label": "cytosol",
  "gene": "UniProtKB:P40818",
  "gene_symbol": "USP8",
  "gene_name": "Ubiquitin carboxyl-terminal hydrolase 8"
}